{
  "term_id": "GO:0006396",
  "gene": "UniProtKB:Q05823",
  "gene_name": "2-5A-dependent ribonuclease",
  "gene_symbol": "RNASEL",
  "term_label": "RNA processing"
}